{
  "term_id": "UNKNOWN:0001",
  "gene_symbol": "CBLN4",
  "term_label": "Unknown molecular function",
  "gene": "UniProtKB:Q9NTU7",
  "gene_name": "Cerebellin-4"
}